{
  "term_label": "cell adhesion",
  "gene_name": "Protocadherin-9",
  "gene_symbol": "PCDH9",
  "gene": "UniProtKB:Q9HC56",
  "term_id": "GO:0007155"
}